{
  "gene": "UniProtKB:P54710",
  "term_id": "UNKNOWN:0003",
  "gene_symbol": "FXYD2",
  "term_label": "Unknown cellular component",
  "gene_name": "Sodium_potassium-transporting ATPase subunit gamma"
}